{
  "term_id": "GO:0031012",
  "gene_name": "von Willebrand factor",
  "term_label": "extracellular matrix",
  "gene_symbol": "VWF",
  "gene": "UniProtKB:P04275"
}